{
  "gene_symbol": "OR1I1",
  "term_label": "olfactory receptor activity",
  "term_id": "GO:0004984",
  "gene_name": "Olfactory receptor 1I1",
  "gene": "UniProtKB:O60431"
}